peripheral nervous system non-myelinated axon ensheathment [GO:0032294] (biological process) Also known as: ensheathment of non-myelinated axons in peripheral nervous system Relationships: is a type of non-myelinated axon ensheathment [GO:0032285]; is a type of peripheral nervous system axon ensheathment [GO:0032292] Sources: GOC:dgh Definition: The process in which a non-myelinating Schwann cell membrane encircles an axon in the peripheral nervous system. A single non-myelinating Schwann cell will typically associate with multiple axons.